11-oxo-beta-amyrin catabolic process [GO:1902382] (biological process) Also known as: 11-oxo-beta-amyrin breakdown, 11-oxo-beta-amyrin catabolism, 11-oxo-beta-amyrin degradation References: PMID:22128119 Sources: GOC:TermGenie Relationships: is a type of pentacyclic triterpenoid catabolic process [GO:0019741]; is a type of GO:0042182 Definition: The chemical reactions and pathways resulting in the breakdown of 11-oxo-beta-amyrin.